{
  "gene": "UniProtKB:Q8N468",
  "gene_symbol": "MFSD4A",
  "term_id": "UNKNOWN:0001",
  "term_label": "Unknown molecular function",
  "gene_name": "Major facilitator superfamily domain-containing protein 4A"
}